{
  "term_label": "regulation of transcription by RNA polymerase II",
  "gene_name": "Lysine-specific demethylase 2A",
  "term_id": "GO:0006357",
  "gene_symbol": "KDM2A",
  "gene": "UniProtKB:Q9Y2K7"
}